{
  "term_label": "Unknown biological process",
  "gene_name": "Ethanolamine-phosphate phospho-lyase",
  "gene_symbol": "ETNPPL",
  "gene": "UniProtKB:Q8TBG4",
  "term_id": "UNKNOWN:0002"
}